oxidoreductase activity, acting on the CH-CH group of donors, quinone or related compound as acceptor [GO:0016635] (molecular function) Relationships: is a type of oxidoreductase activity, acting on the CH-CH group of donors [GO:0016627] Sources: EC:1.3.5.- Subtypes: succinate dehydrogenase (quinone) activity [GO:0008177], 9,9'-di-cis-zeta-carotene desaturase activity [GO:0016719], menaquinone-dependent protoporphyrinogen oxidase activity [GO:0070819], GO:0106430 Definition: Catalysis of an oxidation-reduction (redox) reaction in which a CH-CH group acts as a hydrogen or electron donor and reduces a quinone or related compound.